PET complex [GO:1990923] (cellular component) Definition: A protein complex that is composed of at least EXD1, TDRD12 and some PIWI protein. The complex is required for MILI slicing-triggered biogenesis and loading of MIWI2 piRNAs. Relationships: is_a GO:0032991 References: PMID:26669262 Subtypes: Rhino-Deadlock-Cutoff Complex [GO:1990469]